{
  "term_label": "Unknown biological process",
  "gene_name": "Serpin B5",
  "gene_symbol": "SERPINB5",
  "gene": "UniProtKB:P36952",
  "term_id": "UNKNOWN:0002"
}